{
  "term_id": "GO:0000978",
  "gene_name": "Recombining binding protein suppressor of hairless-like protein",
  "gene_symbol": "RBPJL",
  "gene": "UniProtKB:Q9UBG7",
  "term_label": "RNA polymerase II cis-regulatory region sequence-specific DNA binding"
}